{
  "gene": "UniProtKB:O00186",
  "term_label": "secretory granule",
  "gene_name": "Syntaxin-binding protein 3",
  "gene_symbol": "STXBP3",
  "term_id": "GO:0030141"
}